interleukin-1 receptor binding [GO:0005149] (molecular function) Relationships: is a type of GO:0005126; is a type of growth factor receptor binding [GO:0070851] Sources: GOC:go_curators Definition: Binding to an interleukin-1 receptor. Also known as: IL-1, interleukin-1 receptor ligand Subtypes: GO:0005150, interleukin-1, type II receptor binding [GO:0005151]